{
  "gene_name": "Neuropilin-1",
  "term_id": "GO:0030424",
  "gene": "UniProtKB:O14786",
  "gene_symbol": "NRP1",
  "term_label": "axon"
}